{
  "term_label": "Unknown biological process",
  "gene": "UniProtKB:O95907",
  "gene_name": "Monocarboxylate transporter 3",
  "gene_symbol": "SLC16A8",
  "term_id": "UNKNOWN:0002"
}